{
  "gene_symbol": "GCC1",
  "gene": "UniProtKB:Q96CN9",
  "gene_name": "GRIP and coiled-coil domain-containing protein 1",
  "term_label": "Unknown molecular function",
  "term_id": "UNKNOWN:0001"
}